cellular response to Aroclor 1254 [GO:1904011] (biological process) Definition: Any process that results in a change in state or activity of a cell (in terms of movement, secretion, enzyme production, gene expression, etc.) as a result of an Aroclor 1254 stimulus. Relationships: is a type of cellular response to chemical stimulus [GO:0070887]; is a type of response to Aroclor 1254 [GO:1904010] References: PMID:18602130 Sources: GOC:TermGenie, GO_REF:0000071